negative regulation of potassium ion import across plasma membrane [GO:1903287] (biological process) Relationships: is a type of negative regulation of potassium ion transmembrane transport [GO:1901380]; is a type of regulation of potassium ion import [GO:1903286]; negatively regulates potassium ion import across plasma membrane [GO:1990573] Definition: Any process that stops, prevents or reduces the frequency, rate or extent of potassium ion import across the plasma membrane. References: PMID:10636900 Sources: GOC:BHF, GOC:TermGenie, GOC:mtg_cardiac_conduct_nov11, GOC:rl, GO_REF:0000058 Also known as: down regulation of potassium import, down regulation of potassium ion import, down regulation of potassium ion uptake, down-regulation of potassium import, down-regulation of potassium ion import, down-regulation of potassium ion uptake, downregulation of potassium import, downregulation of potassium ion import, downregulation of potassium ion uptake, negative regulation of potassium import, negative regulation of potassium ion import, negative regulation of potassium ion uptake, inhibition of potassium import, inhibition of potassium ion import, inhibition of potassium ion uptake